{
  "term_id": "GO:0120162",
  "gene": "UniProtKB:P55916",
  "term_label": "positive regulation of cold-induced thermogenesis",
  "gene_symbol": "UCP3",
  "gene_name": "Putative mitochondrial transporter UCP3"
}